{
  "term_id": "UNKNOWN:0003",
  "term_label": "Unknown cellular component",
  "gene_name": "Acidic leucine-rich nuclear phosphoprotein 32 family member D",
  "gene_symbol": "ANP32D",
  "gene": "UniProtKB:O95626"
}